{
  "term_label": "long-chain fatty acid transmembrane transporter activity",
  "gene_name": "ATP-binding cassette sub-family D member 1",
  "term_id": "GO:0005324",
  "gene_symbol": "ABCD1",
  "gene": "UniProtKB:P33897"
}